{
  "term_label": "GTP binding",
  "gene_name": "ADP-ribosylation factor-like protein 1",
  "gene_symbol": "ARL1",
  "term_id": "GO:0005525",
  "gene": "UniProtKB:P40616"
}